{
  "gene": "UniProtKB:Q9P212",
  "term_label": "phosphatidylinositol-4,5-bisphosphate phospholipase C activity",
  "term_id": "GO:0004435",
  "gene_symbol": "PLCE1",
  "gene_name": "1-phosphatidylinositol 4,5-bisphosphate phosphodiesterase epsilon-1"
}